alpha,alpha-trehalose-phosphate synthase (UDP-forming) activity [GO:0003825] (molecular function) Sources: EC:2.4.1.15 Definition: Catalysis of the reaction: UDP-glucose + D-glucose-6-phosphate = UDP + alpha,alpha-trehalose-6-phosphate. Relationships: is a type of UDP-glucosyltransferase activity [GO:0035251] Also known as: UDP-glucose-glucose-phosphate glucosyltransferase activity, UDP-glucose:D-glucose-6-phosphate 1-alpha-D-glucosyltransferase activity, transglucosylase activity, trehalose 6-phosphate synthase activity, trehalose 6-phosphate synthetase activity, trehalose-phosphate synthase activity, trehalose-phosphate synthetase activity, trehalosephosphate-UDP glucosyl transferase activity, trehalosephosphate-UDP glucosyltransferase activity, UDP-glucose-glucosephosphate glucosyltransferase activity, UDPglucose-glucose-phosphate glucosyltransferase activity, UDPglucose:D-glucose-6-phosphate 1-alpha-D-glucosyltransferase activity, alpha,alpha-trehalose phosphate synthase (UDP-forming), phosphotrehalose-uridine diphosphate transglucosylase activity, trehalose phosphate synthase activity, trehalose phosphate synthetase activity, trehalose phosphate-uridine diphosphate glucosyltransferase activity, trehalose-P synthetase activity, uridine diphosphoglucose phosphate glucosyltransferase activity